{
  "gene": "UniProtKB:Q14CM0",
  "gene_symbol": "FRMPD4",
  "term_id": "GO:0043197",
  "term_label": "dendritic spine",
  "gene_name": "FERM and PDZ domain-containing protein 4"
}